muscle thin filament assembly [GO:0071689] (biological process) Sources: GOC:mah Definition: The aggregation, arrangement and bonding together of proteins to form the actin-based thin filaments of myofibrils in striated muscle. Relationships: is_a GO:0007015; is part of myofibril assembly [GO:0030239]